{
  "gene": "UniProtKB:P41182",
  "gene_name": "B-cell lymphoma 6 protein",
  "term_label": "RNA polymerase II cis-regulatory region sequence-specific DNA binding",
  "gene_symbol": "BCL6",
  "term_id": "GO:0000978"
}